{
  "term_id": "GO:0016020",
  "term_label": "membrane",
  "gene": "UniProtKB:Q8NC44",
  "gene_name": "Reticulophagy regulator 2",
  "gene_symbol": "RETREG2"
}